{
  "term_label": "chemokine activity",
  "gene_symbol": "CCL7",
  "gene": "UniProtKB:P80098",
  "gene_name": "C-C motif chemokine 7",
  "term_id": "GO:0008009"
}